{
  "term_id": "GO:0005737",
  "gene_symbol": "KHDC1",
  "gene_name": "KH homology domain-containing protein 1",
  "term_label": "cytoplasm",
  "gene": "UniProtKB:Q4VXA5"
}